{
  "term_id": "GO:0050852",
  "gene": "UniProtKB:Q08881",
  "term_label": "T cell receptor signaling pathway",
  "gene_symbol": "ITK",
  "gene_name": "Tyrosine-protein kinase ITK_TSK"
}